{
  "gene": "UniProtKB:Q6PJ69",
  "gene_name": "E3 ubiquitin-protein ligase TRIM65",
  "term_label": "positive regulation of autophagy",
  "term_id": "GO:0010508",
  "gene_symbol": "TRIM65"
}